{
  "gene": "UniProtKB:Q9NZJ0",
  "term_id": "GO:0030674",
  "gene_symbol": "DTL",
  "term_label": "protein-macromolecule adaptor activity",
  "gene_name": "Denticleless protein homolog"
}